{
  "gene": "UniProtKB:A0A087WW87",
  "term_id": "GO:0019814",
  "term_label": "immunoglobulin complex",
  "gene_name": "Immunoglobulin kappa variable 2-40",
  "gene_symbol": "IGKV2-40"
}